negative regulation of interleukin-13 production [GO:0032696] (biological process) Sources: GOC:mah Also known as: down regulation of interleukin-13 production, down-regulation of interleukin-13 production, downregulation of interleukin-13 production, negative regulation of IL-13 production, inhibition of interleukin-13 production, negative regulation of interleukin-13 biosynthetic process, negative regulation of interleukin-13 secretion Definition: Any process that stops, prevents, or reduces the frequency, rate, or extent of interleukin-13 production. Relationships: is a type of GO:0001818; is_a regulation of interleukin-13 production [GO:0032656]; negatively regulates interleukin-13 production [GO:0032616]